{
  "gene_symbol": "SLC7A4",
  "term_label": "amino acid transmembrane transporter activity",
  "term_id": "GO:0015171",
  "gene": "UniProtKB:O43246",
  "gene_name": "Cationic amino acid transporter 4"
}